RAVE complex [GO:0043291] (cellular component) Definition: A multisubunit complex that in Saccharomyces is composed of three subunits, Rav1p, Rav2p and Skp1p. Acts transiently to catalyze assembly of cytoplasmic V1, with membrane embedded V0 to form the V-ATPase holoenzyme. References: PMID:11283612, PMID:11844802 Also known as: regulator of the (H+)-ATPase of the vacuolar and endosomal membranes Relationships: is a type of protein-containing complex [GO:0032991]; is part of cytoplasm [GO:0005737]